{
  "gene_name": "Max-like protein X",
  "gene_symbol": "MLX",
  "term_id": "GO:0006357",
  "term_label": "regulation of transcription by RNA polymerase II",
  "gene": "UniProtKB:Q9UH92"
}